{
  "gene_name": "Cation channel sperm-associated protein 3",
  "term_label": "sodium ion transport",
  "term_id": "GO:0006814",
  "gene": "UniProtKB:Q86XQ3",
  "gene_symbol": "CATSPER3"
}